{
  "gene_symbol": "S100A16",
  "term_id": "GO:0048471",
  "gene_name": "Protein S100-A16",
  "term_label": "perinuclear region of cytoplasm",
  "gene": "UniProtKB:Q96FQ6"
}